{
  "term_label": "brain-derived neurotrophic factor receptor activity",
  "gene_name": "BDNF_NT-3 growth factors receptor",
  "gene": "UniProtKB:Q16620",
  "term_id": "GO:0060175",
  "gene_symbol": "NTRK2"
}